{
  "gene_name": "Augurin",
  "gene_symbol": "ECRG4",
  "term_label": "anaphase-promoting complex-dependent catabolic process",
  "gene": "UniProtKB:Q9H1Z8",
  "term_id": "GO:0031145"
}